{
  "gene_name": "Tyrosine-protein kinase JAK3",
  "gene": "UniProtKB:P52333",
  "term_label": "cell differentiation",
  "term_id": "GO:0030154",
  "gene_symbol": "JAK3"
}